{
  "term_id": "GO:0034332",
  "gene_name": "Cadherin-8",
  "gene_symbol": "CDH8",
  "gene": "UniProtKB:P55286",
  "term_label": "adherens junction organization"
}